humoral immune response [GO:0006959] (biological process) Sources: GOC:hb, ISBN:0198506732 Regulation: regulated by regulation of humoral immune response [GO:0002920]; negatively regulated by negative regulation of humoral immune response [GO:0002921]; positively regulated by positive regulation of humoral immune response [GO:0002922] Subtypes: humoral immune response mediated by circulating immunoglobulin [GO:0002455], complement activation [GO:0006956], antimicrobial humoral response [GO:0019730], hemolymph coagulation [GO:0042381] Definition: An immune response mediated through a body fluid. Relationships: is a type of immune response [GO:0006955]